{
  "gene_symbol": "UQCRH",
  "term_id": "GO:0006122",
  "gene_name": "Cytochrome b-c1 complex subunit 6, mitochondrial",
  "gene": "UniProtKB:P07919",
  "term_label": "mitochondrial electron transport, ubiquinol to cytochrome c"
}